{
  "term_label": "Unknown molecular function",
  "term_id": "UNKNOWN:0001",
  "gene": "UniProtKB:Q9UL45",
  "gene_name": "Biogenesis of lysosome-related organelles complex 1 subunit 6",
  "gene_symbol": "BLOC1S6"
}